{
  "gene_symbol": "CRACR2B",
  "gene_name": "EF-hand calcium-binding domain-containing protein 4A",
  "term_id": "UNKNOWN:0001",
  "term_label": "Unknown molecular function",
  "gene": "UniProtKB:Q8N4Y2"
}